{
  "gene": "UniProtKB:Q7Z6G3",
  "gene_symbol": "NECAB2",
  "term_label": "regulation of amyloid precursor protein biosynthetic process",
  "term_id": "GO:0042984",
  "gene_name": "N-terminal EF-hand calcium-binding protein 2"
}